regulation of steroid metabolic process [GO:0019218] (biological process) Relationships: is a type of regulation of lipid metabolic process [GO:0019216]; regulates steroid metabolic process [GO:0008202] Definition: Any process that modulates the frequency, rate or extent of the chemical reactions and pathways involving steroids. Also known as: regulation of steroid metabolism Sources: GOC:go_curators Subtypes: regulation of ecdysteroid metabolic process [GO:0007553], regulation of glucocorticoid metabolic process [GO:0031943], GO:0032344, negative regulation of steroid metabolic process [GO:0045939], positive regulation of steroid metabolic process [GO:0045940], regulation of steroid biosynthetic process [GO:0050810], GO:0090181